{
  "term_id": "GO:0005886",
  "term_label": "plasma membrane",
  "gene_symbol": "AQP5",
  "gene_name": "Aquaporin-5",
  "gene": "UniProtKB:P55064"
}